{
  "gene": "UniProtKB:O43315",
  "gene_symbol": "AQP9",
  "term_label": "basolateral plasma membrane",
  "term_id": "GO:0016323",
  "gene_name": "Aquaporin-9"
}